4-amino-4-deoxychorismate synthase activity [GO:0046820] (molecular function) Note: Note that the name 'para-aminobenzoic acid synthase' was initially given to the 'aminodeoxychorismate synthase' activity before the additional 4-amino-4-deoxychorismate lyase activity was discovered. It is the lyase activity that actually produces para-aminobenzoic acid from 4-amino-4-deoxychorismate. Relationships: is a type of transaminase activity [GO:0008483] Sources: EC:2.6.1.85, RHEA:11672 Definition: Catalysis of the reaction: L-glutamine + chorismate = 4-amino-4-deoxychorismate + L-glutamate. It is composed of two enzymatic activities (which may be present on one or two polypeptides); the first is a glutaminase which yields ammonia from glutamine, releasing glutamate. The ammonia is used by the second activity which catalyzes the amination of chorismate to form 4-amino-4-deoxychorismate. Also known as: ADC synthase activity, PabB activity, aminodeoxychorismate synthase activity, chorismate:L-glutamine amido-ligase activity, p-aminobenzoate synthetase, para-aminobenzoic acid (PABA) synthase, para-aminobenzoic acid synthase activity